response to 2,3,7,8-tetrachlorodibenzodioxine [GO:1904612] (biological process) Also known as: response to TCDD, response to dioxin References: PMID:23196670 Sources: GOC:TermGenie, GO_REF:0000071 Relationships: is a type of response to chemical [GO:0042221] Subtypes: cellular response to 2,3,7,8-tetrachlorodibenzodioxine [GO:1904613] Definition: Any process that results in a change in state or activity of a cell or an organism (in terms of movement, secretion, enzyme production, gene expression, etc.) as a result of a 2,3,7,8-tetrachlorodibenzodioxine stimulus.